{
  "gene": "UniProtKB:Q8NEE0",
  "gene_name": "Putative uncharacterized protein KLHL30-AS1",
  "gene_symbol": "KLHL30-AS1",
  "term_id": "UNKNOWN:0002",
  "term_label": "Unknown biological process"
}